{
  "gene": "UniProtKB:Q99569",
  "gene_name": "Plakophilin-4",
  "term_label": "cadherin binding",
  "gene_symbol": "PKP4",
  "term_id": "GO:0045296"
}